C-5 sterol desaturase activity [GO:0000248] (molecular function) Relationships: is a type of sterol desaturase activity [GO:0070704] Definition: Catalysis of the reaction: 5,7,24(28)-ergostatrienol + O2 + NADPH = 5,7,22,24(28)-ergostatetraenol + 2 H2O + NADP+. Also known as: sterol-C5-desaturase activity Sources: GOC:curators